Rpd3L-Expanded complex [GO:0070210] (cellular component) References: PMID:19040720 Sources: GOC:rb Relationships: is a type of histone deacetylase complex [GO:0000118]; is part of nuclear chromosome [GO:0000228]; is part of chromatin [GO:0000785] Also known as: Clr6-LE complex Definition: A protein complex that contains a histone deacetylase and is part of the chromatin remodeling machinery. In Saccharomyces cerevisiae this complex contains the Rpd3p, Sin3p, Ume1p, Pho23p, Sap30p, Sds3p, Cti6p, Rxt2p, Rxt3p, Dep1p, Ume6p, Ash1p, Dot6p, Snt1, Sif2p, Set3p, Hos2p, Tos4p and Tod6p proteins.